positive regulation of single-strand break repair via homologous recombination [GO:1903112] (biological process) Also known as: up regulation of single-strand break repair via homologous recombination, up-regulation of single-strand break repair via homologous recombination, upregulation of single-strand break repair via homologous recombination, activation of single-strand break repair via homologous recombination References: PMID:24339919 Sources: GOC:TermGenie, GOC:bhm, GO_REF:0000058 Relationships: is a type of positive regulation of DNA recombination [GO:0045911]; is a type of regulation of single-strand break repair via homologous recombination [GO:1903110]; is a type of positive regulation of single strand break repair [GO:1903518]; positively regulates single-strand break repair via homologous recombination [GO:1990396] Definition: Any process that activates or increases the frequency, rate or extent of single-strand break repair via homologous recombination.